{
  "gene": "UniProtKB:Q9UNI6",
  "gene_symbol": "DUSP12",
  "term_label": "nucleus",
  "term_id": "GO:0005634",
  "gene_name": "Dual specificity protein phosphatase 12"
}